putamen development [GO:0021758] (biological process) Definition: The progression of the putamen over time from its initial formation until its mature state. The putamen is the lens-shaped basal ganglion involved with control of voluntary movement in the brain. Sources: GOC:cls, GOC:dgh, GOC:dph, GOC:jid, GO_REF:0000021 Relationships: is a type of neural nucleus development [GO:0048857]; is part of GO:0021756